{
  "term_label": "cell morphogenesis",
  "gene_symbol": "CDH1",
  "term_id": "GO:0000902",
  "gene": "UniProtKB:P12830",
  "gene_name": "Cadherin-1"
}